{
  "gene_symbol": "CCNB1",
  "gene": "UniProtKB:P14635",
  "term_id": "GO:0007080",
  "gene_name": "G2_mitotic-specific cyclin-B1",
  "term_label": "mitotic metaphase chromosome alignment"
}